{
  "term_label": "Unknown cellular component",
  "gene_name": "Cell growth regulator with RING finger domain protein 1",
  "term_id": "UNKNOWN:0003",
  "gene_symbol": "CGRRF1",
  "gene": "UniProtKB:Q99675"
}